{
  "gene_symbol": "ADAMTS16",
  "gene_name": "A disintegrin and metalloproteinase with thrombospondin motifs 16",
  "gene": "UniProtKB:Q8TE57",
  "term_id": "GO:0006508",
  "term_label": "proteolysis"
}